{
  "gene_symbol": "C4orf54",
  "term_label": "Unknown biological process",
  "gene_name": "Uncharacterized protein C4orf54",
  "term_id": "UNKNOWN:0002",
  "gene": "UniProtKB:D6RIA3"
}